{
  "gene": "UniProtKB:Q8NH81",
  "term_id": "GO:0004984",
  "gene_name": "Olfactory receptor 10G6",
  "gene_symbol": "OR10G6",
  "term_label": "olfactory receptor activity"
}